{
  "gene_symbol": "IGHV1-18",
  "term_id": "UNKNOWN:0003",
  "gene": "UniProtKB:A0A0C4DH31",
  "term_label": "Unknown cellular component",
  "gene_name": "Immunoglobulin heavy variable 1-18"
}